{
  "gene_symbol": "MAPK12",
  "term_label": "nucleus",
  "gene_name": "Mitogen-activated protein kinase 12",
  "term_id": "GO:0005634",
  "gene": "UniProtKB:P53778"
}